molting cycle process [GO:0022404] (biological process) Subtypes: chitin-based cuticle sclerotization [GO:0007593], apolysis [GO:0018989], ecdysis, chitin-based cuticle [GO:0018990], GO:0022405, collagen and cuticulin-based cuticle attachment to epithelium [GO:0040004], chitin-based cuticle attachment to epithelium [GO:0040005], GO:0042395 Sources: GOC:isa_complete Definition: A multicellular organismal process involved in the periodic casting off and regeneration of an outer covering of cuticle, feathers, hair, horns, skin. Relationships: is a type of multicellular organismal process [GO:0032501]; is part of molting cycle [GO:0042303]